{
  "term_label": "Unknown molecular function",
  "term_id": "UNKNOWN:0001",
  "gene": "UniProtKB:A0A494C0N9",
  "gene_symbol": "FAM246B",
  "gene_name": "Protein FAM246B"
}